{
  "gene_name": "Zinc finger protein 436",
  "term_label": "nucleus",
  "gene": "UniProtKB:Q9C0F3",
  "term_id": "GO:0005634",
  "gene_symbol": "ZNF436"
}